{
  "gene_name": "Tumor necrosis factor receptor superfamily member 1A",
  "term_label": "receptor complex",
  "gene_symbol": "TNFRSF1A",
  "gene": "UniProtKB:P19438",
  "term_id": "GO:0043235"
}